protein tyrosine kinase binding [GO:1990782] (molecular function) Definition: Binding to protein tyrosine kinase. Relationships: is a type of protein kinase binding [GO:0019901] Subtypes: receptor tyrosine kinase binding [GO:0030971] Also known as: tyrosine kinase binding References: PMID:25499537